{
  "term_id": "GO:0032755",
  "gene_symbol": "HSPD1",
  "gene": "UniProtKB:P10809",
  "term_label": "positive regulation of interleukin-6 production",
  "gene_name": "60 kDa heat shock protein, mitochondrial"
}